{
  "term_id": "UNKNOWN:0001",
  "term_label": "Unknown molecular function",
  "gene_name": "Ras-like protein family member 10B",
  "gene_symbol": "RASL10B",
  "gene": "UniProtKB:Q96S79"
}